beta-ribofuranosylaminobenzene 5'-phosphate synthase activity [GO:0043793] (MF) Relationships: is a type of pentosyltransferase activity [GO:0016763] Also known as: beta-RFAP synthase activity References: PMID:12142414 Sources: EC:2.4.2.54 Definition: Catalysis of the reaction: 4-hydroxybenzoate + 5-phospho-alpha-D-ribose 1-diphosphate + H+ = 4-(beta-D-ribofuranosyl)phenol 5'-phosphate + CO2 + diphosphate. Both 4-hydroxybenzoate and 4-aminobenzoate may be used as substrates, but only the former is known to be produced by methanogenic archaea.